citrate-L-glutamate ligase activity [GO:0072591] (molecular function) Relationships: is a type of GO:0016879 References: PMID:20657015 Definition: Catalysis of the reaction: ATP + citrate + L-glutamate = ADP + phosphate + beta-citryl-L-glutamate.